{
  "gene": "UniProtKB:P08185",
  "gene_symbol": "SERPINA6",
  "term_id": "UNKNOWN:0002",
  "term_label": "Unknown biological process",
  "gene_name": "Corticosteroid-binding globulin"
}